viral RNA editing [GO:0075527] (BP) References: PMID:1629949 Sources: VZ:857 Relationships: is a type of viral process [GO:0016032]; is part of viral transcription [GO:0019083] Definition: The process by which bases in viral mRNA are chemically altered during viral transcription. This is usually the incorporation of 1 - 6 additional nucleotides, which shifts the reading frame, allowing the generation of different protein products or through a specific nucleotide change that eliminates the termination codon. Also known as: RNA editing involved in viral mRNA transcription